{
  "gene": "UniProtKB:P0C7A2",
  "gene_name": "Protein FAM153B",
  "term_label": "Unknown cellular component",
  "term_id": "UNKNOWN:0003",
  "gene_symbol": "FAM153B"
}